{
  "gene_name": "Phospholipid scramblase family member 5",
  "gene": "UniProtKB:A0PG75",
  "term_id": "GO:0017121",
  "gene_symbol": "PLSCR5",
  "term_label": "plasma membrane phospholipid scrambling"
}